{
  "term_label": "clathrin adaptor activity",
  "gene_symbol": "AP1M2",
  "gene": "UniProtKB:Q9Y6Q5",
  "gene_name": "AP-1 complex subunit mu-2",
  "term_id": "GO:0035615"
}